{
  "gene_symbol": "SPDL1",
  "gene": "UniProtKB:Q96EA4",
  "term_id": "GO:0034501",
  "gene_name": "Protein Spindly",
  "term_label": "protein localization to kinetochore"
}